hepatocyte growth factor receptor signaling pathway [GO:0048012] (biological process) Sources: GOC:ceb Also known as: HGF receptor signaling pathway, HGF receptor signalling pathway, Met signaling pathway Definition: The series of molecular signals initiated by a ligand binding to a hepatocyte growth factor receptor, and ending with the regulation of a downstream cellular process, e.g. transcription. Relationships: is a type of cell surface receptor protein tyrosine kinase signaling pathway [GO:0007169] Regulation: regulated by regulation of hepatocyte growth factor receptor signaling pathway [GO:1902202]; negatively regulated by negative regulation of hepatocyte growth factor receptor signaling pathway [GO:1902203]; positively regulated by positive regulation of hepatocyte growth factor receptor signaling pathway [GO:1902204]